{
  "gene_symbol": "LUZP6",
  "gene": "UniProtKB:Q538Z0",
  "gene_name": "Leucine zipper protein 6",
  "term_id": "UNKNOWN:0003",
  "term_label": "Unknown cellular component"
}